{
  "gene": "UniProtKB:P28300",
  "term_label": "extracellular space",
  "term_id": "GO:0005615",
  "gene_name": "Protein-lysine 6-oxidase",
  "gene_symbol": "LOX"
}